mitochondrial transcription factor activity [GO:0034246] (MF) Relationships: is a type of transcription regulator activity [GO:0140110]; is part of mitochondrial transcription [GO:0006390]; has part mitochondrial single-subunit type RNA polymerase binding [GO:0001001]; has part mitochondrial promoter sequence-specific DNA binding [GO:0001018]; occurs in mitochondrion [GO:0005739] Also known as: mitochondrial RNA polymerase binding promoter specificity activity, mitochondrial RNA polymerase core promoter proximal region sequence-specific DNA binding transcription factor activity, mitochondrial RNA polymerase core promoter sequence-specific DNA binding transcription factor activity, mitochondrial RNA polymerase transcription factor activity, sequence-specific DNA binding, mitochondrial polymerase transcription factor activity, mitochondrial sequence-specific DNA binding transcription factor activity, mitochondrial transcription initiation factor activity, sequence-specific DNA binding mitochondrial RNA polymerase transcription factor activity, transcription factor activity, mitochondrial RNA polymerase core promoter proximal region sequence-specific binding, transcription factor activity, mitochondrial RNA polymerase core promoter sequence-specific DNA binding, transcription factor activity, mitochondrial proximal promoter sequence-specific binding, mitochondrial DNA-binding transcription factor activity, mitochondrial sequence-specific DNA-binding transcription factor activity, mitochondrial RNA polymerase promoter specificity activity Definition: Interacting with the mitochondrial promoter DNA to modulate transcription by the mitochondrial RNA polymerase. References: PMID:18391175 Sources: GOC:txnOH-2018